AGC codon-amino acid adaptor activity [GO:0033446] (MF) Also known as: serine tRNA Sources: GOC:mah Relationships: is_a triplet codon-amino acid adaptor activity [GO:0030533] Note: Note that in the standard genetic code, AGC codes for serine. Definition: A triplet codon-amino acid adaptor activity that recognizes an AGC codon.